pyridine biosynthetic process [GO:0046220] (biological process) Sources: GOC:ai Also known as: pyridine anabolism, pyridine biosynthesis, pyridine formation, pyridine synthesis Relationships: is a type of GO:0072525 Definition: The chemical reactions and pathways resulting in the formation of pyridine, a nitrogenous base (C5H5N) obtained from the distillation of bone oil or coal tar, and by the decomposition of certain alkaloids, as a colorless liquid with a peculiar pungent odor.